{
  "term_label": "long-chain fatty acid transport",
  "gene_name": "Fatty acid-binding protein 9",
  "gene_symbol": "FABP9",
  "term_id": "GO:0015909",
  "gene": "UniProtKB:Q0Z7S8"
}